{
  "gene_name": "Small glutamine-rich tetratricopeptide repeat-containing protein alpha",
  "term_id": "GO:0006620",
  "gene_symbol": "SGTA",
  "term_label": "post-translational protein targeting to endoplasmic reticulum membrane",
  "gene": "UniProtKB:O43765"
}